{
  "term_id": "GO:0030126",
  "term_label": "COPI vesicle coat",
  "gene_name": "Coatomer subunit gamma-2",
  "gene_symbol": "COPG2",
  "gene": "UniProtKB:Q9UBF2"
}